{
  "gene": "UniProtKB:Q13454",
  "gene_symbol": "TUSC3",
  "gene_name": "Tumor suppressor candidate 3",
  "term_id": "GO:1903830",
  "term_label": "magnesium ion transmembrane transport"
}